undecaprenyl-phosphate glucose phosphotransferase activity [GO:0089702] (molecular function) Definition: Catalysis of the reaction: di-trans,octa-cis-undecaprenyl phosphate + UDP-alpha-D-glucose = alpha-D-glucosyl di-trans,octa-cis-undecaprenyl diphosphate + UMP. Sources: RHEA:28126 Relationships: is a type of GO:0016780